{
  "gene_symbol": "CX3CL1",
  "term_label": "extracellular space",
  "gene": "UniProtKB:P78423",
  "gene_name": "Fractalkine",
  "term_id": "GO:0005615"
}